phosphatidyl-N-methylethanolamine N-methyltransferase activity [GO:0000773] (molecular function) Also known as: PLMT, S-adenosyl-L-methionine:phosphatidyl-N-methylethanolamine N-methyltransferase activity, methyltransferase II, phosphatidyl-N-methylethanolamine methyltransferase activity, phosphatidyl-N-monomethylethanolamine methyltransferase activity, phosphatidylethanolamine methyltransferase I, phosphatidylmonomethylethanolamine methyltransferase activity, phospholipid methyltransferase activity Relationships: is_a N-methyltransferase activity [GO:0008170]; is a type of GO:0008757 Definition: Catalysis of the reaction: S-adenosyl-L-methionine + phosphatidyl-N-methylethanolamine = S-adenosyl-L-homocysteine + phosphatidyl-N-dimethylethanolamine. Also catalyzes the transfer of a further methylgroup, producing phosphatidylcholine. References: PMID:19366698 Sources: EC:2.1.1.71